{
  "term_id": "UNKNOWN:0003",
  "gene_symbol": "TMEM117",
  "term_label": "Unknown cellular component",
  "gene_name": "Transmembrane protein 117",
  "gene": "UniProtKB:Q9H0C3"
}